{
  "term_label": "RNA polymerase II cis-regulatory region sequence-specific DNA binding",
  "gene_name": "Protein c-Fos",
  "term_id": "GO:0000978",
  "gene_symbol": "FOS",
  "gene": "UniProtKB:P01100"
}